{
  "gene_symbol": "VWC2",
  "gene": "UniProtKB:Q2TAL6",
  "term_label": "Unknown molecular function",
  "gene_name": "Brorin",
  "term_id": "UNKNOWN:0001"
}